{
  "term_label": "endosome",
  "gene": "UniProtKB:Q7Z3J2",
  "gene_name": "VPS35 endosomal protein-sorting factor-like",
  "term_id": "GO:0005768",
  "gene_symbol": "VPS35L"
}